{
  "term_id": "UNKNOWN:0003",
  "gene_name": "BTB_POZ domain-containing protein 19",
  "gene": "UniProtKB:C9JJ37",
  "gene_symbol": "BTBD19",
  "term_label": "Unknown cellular component"
}